{
  "gene_name": "Ras-associated and pleckstrin homology domains-containing protein 1",
  "term_label": "cytosol",
  "gene": "UniProtKB:Q70E73",
  "gene_symbol": "RAPH1",
  "term_id": "GO:0005829"
}